{
  "term_label": "Unknown cellular component",
  "term_id": "UNKNOWN:0003",
  "gene_symbol": "BAGE4",
  "gene": "UniProtKB:Q86Y28",
  "gene_name": "B melanoma antigen 4"
}